{
  "gene": "UniProtKB:Q8WTV1",
  "gene_name": "THAP domain-containing protein 3",
  "gene_symbol": "THAP3",
  "term_label": "Unknown cellular component",
  "term_id": "UNKNOWN:0003"
}